{
  "term_label": "Unknown biological process",
  "gene_name": "Tubulin--tyrosine ligase-like protein 12",
  "term_id": "UNKNOWN:0002",
  "gene_symbol": "TTLL12",
  "gene": "UniProtKB:Q14166"
}